{
  "gene_name": "Cleavage stimulation factor subunit 2 tau variant",
  "gene": "UniProtKB:Q9H0L4",
  "term_label": "mRNA binding",
  "term_id": "GO:0003729",
  "gene_symbol": "CSTF2T"
}